{
  "term_label": "UDP phosphatase activity",
  "gene_name": "Ectonucleoside triphosphate diphosphohydrolase 2",
  "gene": "UniProtKB:Q9Y5L3",
  "gene_symbol": "ENTPD2",
  "term_id": "GO:0045134"
}